{
  "gene_name": "Sodium-coupled neutral amino acid transporter 3",
  "gene": "UniProtKB:Q99624",
  "gene_symbol": "SLC38A3",
  "term_label": "amino acid transmembrane transport",
  "term_id": "GO:0003333"
}